{
  "gene": "UniProtKB:Q9H461",
  "gene_symbol": "FZD8",
  "term_label": "Wnt receptor activity",
  "gene_name": "Frizzled-8",
  "term_id": "GO:0042813"
}